microtubule anchoring at centrosome [GO:0034454] (biological process) Regulation: regulated by regulation of microtubule anchoring at centrosome [GO:0150101] Definition: Any process in which a microtubule is maintained in a specific location in a cell by attachment to a centrosome. Relationships: is_a microtubule anchoring at microtubule organizing center [GO:0072393] Sources: GOC:BHF, GOC:mah